{
  "term_id": "GO:0006612",
  "gene_symbol": "ZDHHC7",
  "gene_name": "Palmitoyltransferase ZDHHC7",
  "term_label": "protein targeting to membrane",
  "gene": "UniProtKB:Q9NXF8"
}